renal inner medulla development [GO:0072053] (biological process) Relationships: is a type of anatomical structure development [GO:0048856]; is part of kidney development [GO:0001822] Also known as: inner renal medulla development Sources: GOC:mtg_kidney_jan10 Definition: The process whose specific outcome is the progression of the renal inner medulla over time, from its formation to the mature structure. The renal inner medulla is unique to mammalian kidneys and is the innermost region of the mammalian kidney.